{
  "gene": "UniProtKB:Q14749",
  "term_id": "GO:0006730",
  "gene_name": "Glycine N-methyltransferase",
  "gene_symbol": "GNMT",
  "term_label": "one-carbon metabolic process"
}